{
  "gene": "UniProtKB:Q8NCW5",
  "gene_name": "NAD(P)H-hydrate epimerase",
  "term_label": "mitochondrion",
  "gene_symbol": "NAXE",
  "term_id": "GO:0005739"
}